{
  "gene": "UniProtKB:Q13216",
  "gene_symbol": "ERCC8",
  "term_label": "Cul4A-RING E3 ubiquitin ligase complex",
  "term_id": "GO:0031464",
  "gene_name": "DNA excision repair protein ERCC-8"
}